{
  "term_label": "adenylate cyclase-activating G protein-coupled receptor signaling pathway",
  "gene": "UniProtKB:Q8WXD0",
  "gene_symbol": "RXFP2",
  "term_id": "GO:0007189",
  "gene_name": "Relaxin receptor 2"
}